{
  "gene_symbol": "RASAL3",
  "gene_name": "RAS protein activator like-3",
  "term_label": "Unknown cellular component",
  "gene": "UniProtKB:Q86YV0",
  "term_id": "UNKNOWN:0003"
}